{
  "gene_symbol": "KLHL36",
  "term_label": "ubiquitin-like ligase-substrate adaptor activity",
  "gene_name": "Kelch-like protein 36",
  "gene": "UniProtKB:Q8N4N3",
  "term_id": "GO:1990756"
}